protein targeting to ER [GO:0045047] (biological process) Definition: The process of directing proteins towards the endoplasmic reticulum (ER) using signals contained within the protein. One common mechanism uses a 16- to 30-residue signal sequence, typically located at the N-terminus of the protein and containing positively charged amino acids followed by a continuous stretch of hydrophobic residues, which directs the ribosome to the ER membrane and initiates transport of the growing polypeptide across the ER membrane. Sources: ISBN:0716731363 Also known as: protein targeting to endoplasmic reticulum, protein-ER targeting, protein-endoplasmic reticulum targeting Relationships: is a type of protein targeting [GO:0006605]; is a type of GO:0072599 Subtypes: GO:0006614, post-translational protein targeting to endoplasmic reticulum membrane [GO:0006620]